{
  "gene_symbol": "SERPINF1",
  "gene_name": "Pigment epithelium-derived factor",
  "term_label": "serine-type endopeptidase inhibitor activity",
  "gene": "UniProtKB:P36955",
  "term_id": "GO:0004867"
}